{
  "gene_symbol": "KCNB1",
  "term_label": "potassium ion transmembrane transport",
  "gene_name": "Potassium voltage-gated channel subfamily B member 1",
  "term_id": "GO:0071805",
  "gene": "UniProtKB:Q14721"
}